{
  "term_label": "replication fork processing",
  "gene": "UniProtKB:Q96HA7",
  "gene_symbol": "TONSL",
  "gene_name": "Tonsoku-like protein",
  "term_id": "GO:0031297"
}